{
  "gene_name": "mRNA export factor GLE1",
  "gene_symbol": "GLE1",
  "gene": "UniProtKB:Q53GS7",
  "term_id": "GO:0044614",
  "term_label": "nuclear pore cytoplasmic filaments"
}